{
  "term_label": "plasma membrane",
  "term_id": "GO:0005886",
  "gene_symbol": "ABCC4",
  "gene_name": "ATP-binding cassette sub-family C member 4",
  "gene": "UniProtKB:O15439"
}